ventral furrow formation [GO:0007370] (biological process) Sources: ISBN:0879694238 Relationships: is a type of anatomical structure formation involved in morphogenesis [GO:0048646]; is part of gastrulation involving germ band extension [GO:0010004] Definition: Formation of a ventral indentation (furrow) from the blastoderm epithelium, which is internalized to form a tube in the interior of the embryo, marking the start of gastrulation.